{
  "term_id": "GO:0000981",
  "gene": "UniProtKB:Q96SC8",
  "gene_symbol": "DMRTA2",
  "gene_name": "Doublesex- and mab-3-related transcription factor A2",
  "term_label": "DNA-binding transcription factor activity, RNA polymerase II-specific"
}